{
  "gene_symbol": "BIRC8",
  "gene": "UniProtKB:Q96P09",
  "term_label": "cytoplasm",
  "term_id": "GO:0005737",
  "gene_name": "Baculoviral IAP repeat-containing protein 8"
}